{
  "gene_name": "Harmonin-binding protein USHBP1",
  "term_label": "Unknown molecular function",
  "gene_symbol": "USHBP1",
  "term_id": "UNKNOWN:0001",
  "gene": "UniProtKB:Q8N6Y0"
}